aldose sugar dehydrogenase activity [GO:0103040] (molecular function) Definition: Catalysis of the reaction: H2O + an aldose + an oxidized electron acceptor = H+ + an aldonate + a reduced electron acceptor. Relationships: is_a oxidoreductase activity, acting on the CH-OH group of donors, quinone or similar compound as acceptor [GO:0016901] References: PMID:16864586 Sources: GOC:pz, MetaCyc:RXN0-6371